{
  "term_id": "GO:0016192",
  "gene_name": "AP-3 complex subunit beta-2",
  "gene_symbol": "AP3B2",
  "term_label": "vesicle-mediated transport",
  "gene": "UniProtKB:Q13367"
}